{
  "term_label": "Unknown cellular component",
  "gene": "UniProtKB:Q96FA3",
  "gene_symbol": "PELI1",
  "term_id": "UNKNOWN:0003",
  "gene_name": "E3 ubiquitin-protein ligase pellino homolog 1"
}